female gonad morphogenesis [GO:0061040] (biological process) Also known as: ovary morphogenesis Relationships: is a type of GO:0035262; is part of female gonad development [GO:0008585] Definition: The process in which a female gonad is generated and organized. Sources: GOC:BHF, GOC:dph